negative regulation of actin filament annealing [GO:0110055] (biological process) Definition: Any process that stops, prevents or reduces the frequency, rate or extent of actin filament annealing, i.e. the end-to-end joining of existing actin filaments. References: PMID:15743909 Sources: GOC:mah Relationships: is_a GO:0110054